{
  "term_label": "nucleus",
  "gene": "UniProtKB:Q9NTX7",
  "gene_name": "E3 ubiquitin-protein ligase RNF146",
  "term_id": "GO:0005634",
  "gene_symbol": "RNF146"
}